{
  "gene_name": "T cell receptor gamma variable 5",
  "gene": "UniProtKB:A0A0B4J1U4",
  "term_label": "Unknown cellular component",
  "gene_symbol": "TRGV5",
  "term_id": "UNKNOWN:0003"
}